{
  "term_label": "proteasome-mediated ubiquitin-dependent protein catabolic process",
  "gene_symbol": "WWP1",
  "gene": "UniProtKB:Q9H0M0",
  "term_id": "GO:0043161",
  "gene_name": "NEDD4-like E3 ubiquitin-protein ligase WWP1"
}